PNGase complex [GO:0120125] (cellular component) Definition: A protein complex responsible for the catalysis of the reaction: 4-N-(N-acetyl-D-glucosaminyl)-protein + H2O = N-acetyl-beta-D-glucosaminylamine + peptide L-aspartate. This reaction is the hydrolysis of an N4-(acetyl-beta-D-glucosaminyl)asparagine residue in which the N-acetyl-D-glucosamine residue may be further glycosylated, to yield a (substituted) N-acetyl-beta-D-glucosaminylamine and the peptide containing an aspartic residue. References: PMID:15964983, PMID:16249333 Sources: GOC:lnp Relationships: is a type of peptidase complex [GO:1905368]